{
  "term_label": "nucleus",
  "gene_symbol": "PPM1E",
  "gene": "UniProtKB:Q8WY54",
  "gene_name": "Protein phosphatase 1E",
  "term_id": "GO:0005634"
}